{
  "term_label": "actin cytoskeleton organization",
  "gene": "UniProtKB:P53814",
  "gene_symbol": "SMTN",
  "term_id": "GO:0030036",
  "gene_name": "Smoothelin"
}